{
  "term_id": "GO:0004984",
  "gene": "UniProtKB:Q9UGF7",
  "term_label": "olfactory receptor activity",
  "gene_symbol": "OR12D3",
  "gene_name": "Olfactory receptor 12D3"
}